{
  "gene_name": "Interleukin-5",
  "term_label": "extracellular space",
  "term_id": "GO:0005615",
  "gene_symbol": "IL5",
  "gene": "UniProtKB:P05113"
}